{
  "term_id": "GO:0006338",
  "gene_symbol": "PBRM1",
  "gene": "UniProtKB:Q86U86",
  "term_label": "chromatin remodeling",
  "gene_name": "Protein polybromo-1"
}